{
  "gene": "UniProtKB:P30044",
  "gene_name": "Peroxiredoxin-5, mitochondrial",
  "term_id": "GO:0045454",
  "term_label": "cell redox homeostasis",
  "gene_symbol": "PRDX5"
}